positive regulation of adult somatic muscle development [GO:0062227] (biological process) References: PMID:16643882, PMID:25758712 Definition: Any process that increases the rate, frequency or extent of adult somatic muscle development. Relationships: is a type of GO:0062224; is a type of regulation of adult somatic muscle development [GO:0062226]; positively regulates adult somatic muscle development [GO:0007527]